{
  "gene_name": "Transmembrane glycoprotein NMB",
  "gene_symbol": "GPNMB",
  "gene": "UniProtKB:Q14956",
  "term_id": "GO:0007155",
  "term_label": "cell adhesion"
}